{
  "term_id": "GO:0000976",
  "gene_name": "Zinc finger protein 507",
  "term_label": "transcription cis-regulatory region binding",
  "gene": "UniProtKB:Q8TCN5",
  "gene_symbol": "ZNF507"
}